{
  "gene": "UniProtKB:Q9BXR5",
  "gene_name": "Toll-like receptor 10",
  "term_label": "inflammatory response",
  "term_id": "GO:0006954",
  "gene_symbol": "TLR10"
}